{
  "gene": "UniProtKB:Q8IXK2",
  "gene_name": "Polypeptide N-acetylgalactosaminyltransferase 12",
  "gene_symbol": "GALNT12",
  "term_label": "polypeptide N-acetylgalactosaminyltransferase activity",
  "term_id": "GO:0004653"
}